{
  "gene_symbol": "RGPD8",
  "gene_name": "RANBP2-like and GRIP domain-containing protein 8",
  "term_label": "nuclear export",
  "gene": "UniProtKB:O14715",
  "term_id": "GO:0051168"
}